protein-L-isoaspartate (D-aspartate) O-methyltransferase activity [GO:0004719] (molecular function) Definition: Catalysis of the reaction: S-adenosyl-L-methionine + protein L-beta-aspartate = S-adenosyl-L-homocysteine + protein L-beta-aspartate methyl ester. Relationships: is a type of S-adenosylmethionine-dependent methyltransferase activity [GO:0008757]; is a type of protein carboxyl O-methyltransferase activity [GO:0051998] Also known as: D-aspartyl/L-isoaspartyl methyltransferase activity, L-aspartyl/L-isoaspartyl protein methyltransferase activity, L-isoaspartyl protein carboxyl methyltransferase activity, L-isoaspartyl/D-aspartyl protein carboxyl methyltransferase activity, S-adenosyl-L-methionine:protein-L-isoaspartate O-methyltransferase activity, protein (D-aspartate) methyltransferase activity, protein D-aspartate methyltransferase activity, protein L-isoaspartate methyltransferase activity, protein L-isoaspartyl methyltransferase activity, protein O-methyltransferase (L-isoaspartate), protein beta-aspartate O-methyltransferase activity, protein-L-isoaspartate O-methyltransferase activity, protein-L-isoaspartate(D-aspartate) O-methyltransferase activity, protein-beta-aspartate O-methyltransferase activity Sources: EC:2.1.1.77